arachidonate secretion [GO:0050482] (biological process) Definition: The controlled release of arachidonic acid from a cell or a tissue. Relationships: is a type of icosanoid secretion [GO:0032309]; is a type of arachidonate transport [GO:1903963] Also known as: arachidonic acid secretion Note: This term should be used to annotate release of arachidonic acid from the cell. For the hydrolytic release of arachidonic acid from a phospholipid, consider instead annotating to 'phospholipase A2 activity ; GO:0004623'. Regulation: regulated by regulation of arachidonate secretion [GO:0090237]; positively regulated by positive regulation of arachidonate secretion [GO:0090238]; negatively regulated by GO:1900139 Sources: GOC:ai